{
  "term_id": "GO:0098978",
  "gene_symbol": "PCDH9",
  "gene": "UniProtKB:Q9HC56",
  "gene_name": "Protocadherin-9",
  "term_label": "glutamatergic synapse"
}